{
  "term_id": "GO:0007165",
  "gene": "UniProtKB:P60953",
  "gene_symbol": "CDC42",
  "term_label": "signal transduction",
  "gene_name": "Cell division control protein 42 homolog"
}